{
  "gene": "UniProtKB:Q9BXC0",
  "gene_symbol": "HCAR1",
  "gene_name": "Hydroxycarboxylic acid receptor 1",
  "term_id": "GO:0007186",
  "term_label": "G protein-coupled receptor signaling pathway"
}